spindle midzone [GO:0051233] (cellular component) References: PMID:15296749 Sources: GOC:ai Also known as: central spindle, spindle equator Subtypes: mitotic spindle midzone [GO:1990023], meiotic spindle midzone [GO:1990385] Definition: The area in the center of the spindle where the spindle microtubules from opposite poles overlap. Relationships: is a type of cellular anatomical structure [GO:0110165]; is part of spindle [GO:0005819]